{
  "gene": "UniProtKB:Q9Y5G3",
  "term_label": "plasma membrane",
  "gene_name": "Protocadherin gamma-B1",
  "term_id": "GO:0005886",
  "gene_symbol": "PCDHGB1"
}